thylakoid membrane organization [GO:0010027] (BP) Subtypes: GO:0010547 Definition: A process that is carried out at the cellular level which results in the assembly, arrangement of constituent parts, or disassembly of the thylakoid membrane. Sources: GOC:dph, GOC:jl, GOC:mah, GOC:tb Relationships: is a type of plastid membrane organization [GO:0009668] Note: See also the cellular component term 'thylakoid membrane ; GO:0042651'. Also known as: thylakoid membrane organisation, thylakoid membrane organization and biogenesis